deoxyribonucleotide metabolic process [GO:0009262] (biological process) Sources: GOC:go_curators, ISBN:0198506732 Subtypes: deoxyribonucleotide biosynthetic process [GO:0009263], deoxyribonucleotide catabolic process [GO:0009264], 2'-deoxyribonucleotide metabolic process [GO:0009394] Definition: The chemical reactions and pathways involving a deoxyribonucleotide, a compound consisting of deoxyribonucleoside (a base linked to a deoxyribose sugar) esterified with a phosphate group at either the 3' or 5'-hydroxyl group of the sugar. Relationships: is a type of nucleotide metabolic process [GO:0009117]; is a type of carbohydrate derivative metabolic process [GO:1901135] Also known as: deoxyribonucleotide metabolism